{
  "gene_symbol": "NCOA1",
  "gene_name": "Nuclear receptor coactivator 1",
  "term_label": "nuclear receptor binding",
  "gene": "UniProtKB:Q15788",
  "term_id": "GO:0016922"
}